{
  "gene_symbol": "ARNT2",
  "gene": "UniProtKB:Q9HBZ2",
  "gene_name": "Aryl hydrocarbon receptor nuclear translocator 2",
  "term_label": "DNA-binding transcription factor activity, RNA polymerase II-specific",
  "term_id": "GO:0000981"
}